glutamine-scyllo-inositol transaminase activity [GO:0047310] (molecular function) Also known as: glutamine-scyllo-inosose aminotransferase activity, glutamine-scyllo-inosose transaminase activity, L-glutamine-keto-scyllo-inositol aminotransferase activity, L-glutamine-scyllo-inosose transaminase activity, L-glutamine:2,4,6/3,5-pentahydroxycyclohexanone aminotransferase activity, glutamine scyllo-inosose aminotransferase activity, glutamine--scyllo-inosose aminotransferase activity, glutamine--scyllo-inosose transaminase activity Relationships: is a type of L-glutamine aminotransferase activity [GO:0070548] Definition: Catalysis of the reaction: 2,4,6/3,5-pentahydroxycyclohexanone + L-glutamine = 1-amino-1-deoxy-scyllo-inositol + 2-oxoglutaramate. Sources: EC:2.6.1.50, RHEA:22920